{
  "term_label": "DNA damage response",
  "gene_symbol": "PPP4R3A",
  "term_id": "GO:0006974",
  "gene_name": "Serine_threonine-protein phosphatase 4 regulatory subunit 3A",
  "gene": "UniProtKB:Q6IN85"
}